GDP-L-fucose biosynthetic process [GO:0042350] (biological process) Sources: GOC:jl Also known as: GDP-L-fucose anabolism, GDP-L-fucose biosynthesis, GDP-L-fucose formation, GDP-L-fucose synthesis Subtypes: 'de novo' GDP-L-fucose biosynthetic process [GO:0042351], GDP-L-fucose salvage [GO:0042352] Relationships: is a type of nucleotide-sugar biosynthetic process [GO:0009226]; is a type of GDP-L-fucose metabolic process [GO:0046368] Definition: The chemical reactions and pathways resulting in the formation of GDP-L-fucose, a substance composed of L-fucose in glycosidic linkage with guanosine diphosphate.